{
  "gene": "UniProtKB:Q8TAD2",
  "term_id": "GO:0005615",
  "gene_symbol": "IL17D",
  "term_label": "extracellular space",
  "gene_name": "Interleukin-17D"
}